{
  "gene_symbol": "TPD52",
  "term_id": "GO:0030183",
  "gene": "UniProtKB:P55327",
  "term_label": "B cell differentiation",
  "gene_name": "Tumor protein D52"
}